{
  "term_label": "Unknown molecular function",
  "gene_name": "Brain and acute leukemia cytoplasmic protein",
  "term_id": "UNKNOWN:0001",
  "gene": "UniProtKB:Q8WXS3",
  "gene_symbol": "BAALC"
}